{
  "gene_symbol": "HELZ",
  "gene": "UniProtKB:P42694",
  "term_id": "GO:0043186",
  "term_label": "P granule",
  "gene_name": "Probable helicase with zinc finger domain"
}